{
  "term_label": "regulation of blood pressure",
  "gene_name": "Leucyl-cystinyl aminopeptidase",
  "gene": "UniProtKB:Q9UIQ6",
  "gene_symbol": "LNPEP",
  "term_id": "GO:0008217"
}